{
  "term_id": "GO:0031267",
  "term_label": "small GTPase binding",
  "gene_name": "Coiled-coil domain-containing protein 186",
  "gene_symbol": "CCDC186",
  "gene": "UniProtKB:Q7Z3E2"
}